{
  "term_label": "integrin alpha5-beta1 complex",
  "gene_symbol": "ITGA5",
  "gene_name": "Integrin alpha-5",
  "gene": "UniProtKB:P08648",
  "term_id": "GO:0034674"
}